{
  "term_label": "acetylcholine receptor signaling pathway",
  "gene_symbol": "CHRNB2",
  "gene_name": "Neuronal acetylcholine receptor subunit beta-2",
  "gene": "UniProtKB:P17787",
  "term_id": "GO:0095500"
}